insulin receptor recycling [GO:0038020] (biological process) Relationships: is a type of receptor recycling [GO:0001881]; is part of GO:0046628 References: PMID:3907718 Sources: GOC:bf, GOC:signaling Definition: The process that results in the return of an insulin receptor to an active state at the plasma membrane. An active state is when the receptor is ready to receive an insulin signal. Internalized insulin receptors can be recycled to the plasma membrane or sorted to lysosomes for protein degradation.